{
  "term_id": "GO:0005829",
  "gene_name": "CAD protein",
  "gene_symbol": "CAD",
  "term_label": "cytosol",
  "gene": "UniProtKB:P27708"
}